{
  "term_id": "UNKNOWN:0001",
  "gene": "UniProtKB:A0A2R8YCJ5",
  "gene_symbol": "SMIM41",
  "term_label": "Unknown molecular function",
  "gene_name": "Small integral membrane protein 41"
}